{
  "gene_name": "Kinase D-interacting substrate of 220 kDa",
  "gene": "UniProtKB:Q9ULH0",
  "gene_symbol": "KIDINS220",
  "term_id": "GO:0038180",
  "term_label": "nerve growth factor signaling pathway"
}